ER-to-endosome phospholipid transfer complex [GO:0140622] (cellular component) Definition: Lipid transfer complex that is responsible for the non-vesicular transport of phospholipids, such as phosphatidylserine, from the endoplasmic reticulum to the endosome. It resides in the endosomal (acceptor) membrane and binds to specific lipids on the donor membrane at the ER-endosome contact site. References: PMID:20016005, PMID:24366873 Sources: GOC:lnp Relationships: is a type of membrane protein complex [GO:0098796]; is part of endosome membrane [GO:0010008]